{
  "term_id": "GO:0048471",
  "gene_name": "Ran GTPase-activating protein 1",
  "gene_symbol": "RANGAP1",
  "gene": "UniProtKB:P46060",
  "term_label": "perinuclear region of cytoplasm"
}